{
  "gene": "UniProtKB:Q9Y2H2",
  "term_label": "phosphatidylinositol dephosphorylation",
  "term_id": "GO:0046856",
  "gene_symbol": "INPP5F",
  "gene_name": "Phosphatidylinositide phosphatase SAC2"
}